negative regulation of hh target transcription factor activity [GO:1990787] (biological process) Also known as: negative regulation of hedgehog target transcription factor Definition: Any process that decreases the activity of a transcription factor that activates transcription of Hedgehog-target genes in response to Smoothened signaling. In Drosophila, Cubitus interruptus (Ci) is the only identified transcription factor so far in the Hedgehog signaling pathway. In vertebrates members of the Gli protein family are activated by Hedgehog signaling. References: PMID:24311597 Sources: GOC:bhm Relationships: is a type of negative regulation of smoothened signaling pathway [GO:0045879]; is a type of regulation of DNA-binding transcription factor activity [GO:0051090]